negative regulation of premature acrosome loss [GO:0061950] (biological process) Also known as: negative regulation of spontaneous acrosome loss References: PMID:22228629, PMID:23430248 Definition: Any process that stops, prevents or reduces the discharge, by sperm, of a single, anterior secretory granule before the sperm reaches to the zona pellucida of the oocyte. The process begins with the fusion of the outer acrosomal membrane with the sperm plasma membrane and ends with the exocytosis of the acrosomal contents. Relationships: is a type of regulation of premature acrosome loss [GO:0061949]; is a type of negative regulation of reproductive process [GO:2000242]; negatively regulates premature acrosome loss [GO:0061948]